resolution of DNA recombination intermediates [GO:0071139] (BP) Also known as: resolution of recombination intermediates Sources: GOC:elh, GOC:mah, GOC:vw Definition: The cleavage and rejoining of intermediates, such as Holliday junctions, formed during DNA recombination to produce two intact molecules in which genetic material has been exchanged. Relationships: is a type of DNA metabolic process [GO:0006259]; is part of DNA recombination [GO:0006310] Subtypes: resolution of mitotic recombination intermediates [GO:0071140]